undecaprenyldiphospho-muramoylpentapeptide beta-N-acetylglucosaminyltransferase activity [GO:0050511] (molecular function) Definition: Catalysis of the reaction: Mur2Ac(oyl-L-Ala-gamma-D-Glu-L-Lys-D-Ala-D-Ala)-di-trans,octa-cis-undecaprenyl diphosphate + UDP-N-acetyl-alpha-D-glucosamine = beta-D-GlcNAc-(1->4)-Mur2Ac(oyl-L-Ala-gamm-D-Glu-L-Lys-D-Ala-D-Ala)-di-trans,octa-cis-undecaprenyl diphosphate + H+ + UDP. Sources: RHEA:23192 Also known as: undecaprenyldiphospho-muramoylpentapeptide b-N-acetylglucosaminyltransferase activity, MurG transferase activity, UDP-N-acetyl-D-glucosamine:N-acetyl-alpha-D-muramyl(oyl-L-Ala- gamma-D-Glu-L-Lys-D-Ala-D-Ala)-diphosphoundecaprenol beta-1,4-N-acetylglucosaminlytransferase activity, UDP-N-acetylglucosamine--N-acetylmuramyl-(pentapeptide) pyrophosphoryl-undecaprenol N-acetylglucosamine transferase activity, undecaprenyl-PP-MurNAc-pentapeptide-UDPGlcNAc GlcNAc transferase activity Relationships: is a type of acetylglucosaminyltransferase activity [GO:0008375]